{
  "term_id": "GO:0120230",
  "gene": "UniProtKB:Q9P2W1",
  "gene_name": "Homologous-pairing protein 2 homolog",
  "gene_symbol": "PSMC3IP",
  "term_label": "recombinase activator activity"
}